{
  "term_label": "double-stranded RNA adenosine deaminase activity",
  "gene": "UniProtKB:P78563",
  "gene_name": "Double-stranded RNA-specific editase 1",
  "gene_symbol": "ADARB1",
  "term_id": "GO:0003726"
}